{
  "term_label": "Unknown biological process",
  "term_id": "UNKNOWN:0002",
  "gene_name": "Neurotensin_neuromedin N",
  "gene_symbol": "NTS",
  "gene": "UniProtKB:P30990"
}